microgametogenesis [GO:0055046] (biological process) Sources: GOC:mtg_plant Definition: The process whose specific outcome is the progression of the pollen grain over time, from its formation as the microspore to the mature structure. Relationships: is a type of multicellular organismal process [GO:0032501]; is part of pollen development [GO:0009555] Also known as: pollen development from the microspore